{
  "gene": "UniProtKB:A0A075B6S5",
  "term_id": "GO:0019814",
  "term_label": "immunoglobulin complex",
  "gene_symbol": "IGKV1-27",
  "gene_name": "Immunoglobulin kappa variable 1-27"
}